{
  "gene": "UniProtKB:Q14807",
  "term_id": "GO:0016887",
  "gene_name": "Kinesin-like protein KIF22",
  "term_label": "ATP hydrolysis activity",
  "gene_symbol": "KIF22"
}